{
  "gene_symbol": "TRIM38",
  "gene": "UniProtKB:O00635",
  "term_id": "GO:0046596",
  "term_label": "regulation of viral entry into host cell",
  "gene_name": "E3 ubiquitin-protein ligase TRIM38"
}